rhoptry neck [GO:1990225] (cellular component) Relationships: is a type of cellular anatomical structure [GO:0110165]; is part of rhoptry [GO:0020008] References: PMID:23499754, PMID:23937520, PMID:24002067, PMID:24070999 Sources: GOC:giardia, GOC:pr Definition: Narrow, electron-dense part of the rhoptry that extends through the conoid at the apical tip of an apicomplexan parasite. The rhoptry neck serves as a duct through which the contents of the rhoptry are secreted after attachment to the host has been completed and at the commencement of invasion.